glycoprotein O-fatty-acyltransferase activity [GO:0047965] (molecular function) Sources: EC:2.3.1.142, MetaCyc:GLYCOPROTEIN-O-FATTY-ACYLTRANSFERASE-RXN Relationships: is a type of O-palmitoyltransferase activity [GO:0016416]; is a type of GO:0140103 Definition: Catalysis of the reaction: palmitoyl-CoA + mucus glycoprotein = CoA + O-palmitoylglycoprotein. Also known as: fatty-acyl-CoA:mucus-glycoprotein fatty-acyltransferase activity, protein acyltransferase activity